{
  "term_id": "GO:0000165",
  "gene": "UniProtKB:P36507",
  "term_label": "MAPK cascade",
  "gene_symbol": "MAP2K2",
  "gene_name": "Dual specificity mitogen-activated protein kinase kinase 2"
}